{
  "gene": "UniProtKB:P0C866",
  "term_id": "UNKNOWN:0001",
  "gene_name": "Putative uncharacterized protein encoded by LINC00869",
  "term_label": "Unknown molecular function",
  "gene_symbol": "LINC00869"
}